{
  "term_label": "endomembrane system",
  "term_id": "GO:0012505",
  "gene_name": "Syntaxin-2",
  "gene": "UniProtKB:P32856",
  "gene_symbol": "STX2"
}